{
  "gene": "UniProtKB:P49796",
  "term_id": "UNKNOWN:0002",
  "gene_name": "Regulator of G-protein signaling 3",
  "term_label": "Unknown biological process",
  "gene_symbol": "RGS3"
}